{
  "gene_name": "Zinc fingers and homeoboxes protein 1",
  "term_id": "GO:0006357",
  "gene": "UniProtKB:Q9UKY1",
  "gene_symbol": "ZHX1",
  "term_label": "regulation of transcription by RNA polymerase II"
}